mammary gland epithelial cell proliferation [GO:0033598] (biological process) Relationships: is a type of epithelial cell proliferation [GO:0050673]; is part of mammary gland epithelium development [GO:0061180] Subtypes: epithelial cell proliferation involved in mammary gland bud elongation [GO:0060650], epithelial cell proliferation involved in mammary gland duct elongation [GO:0060750] Regulation: RO_0002211 by GO:0033599; negatively regulated by GO:0033600; positively regulated by GO:0033601 Definition: The multiplication or reproduction of mammary gland epithelial cells, resulting in the expansion of a cell population. Mammary gland epithelial cells make up the covering of surfaces of the mammary gland. The mammary gland is a large compound sebaceous gland that in female mammals is modified to secrete milk. Sources: GOC:dph, GOC:mah